{
  "gene_symbol": "MPP4",
  "term_id": "GO:0005912",
  "gene": "UniProtKB:Q96JB8",
  "gene_name": "MAGUK p55 subfamily member 4",
  "term_label": "adherens junction"
}